{
  "gene_name": "Transmembrane O-methyltransferase",
  "gene_symbol": "TOMT",
  "term_label": "developmental process",
  "term_id": "GO:0032502",
  "gene": "UniProtKB:Q8WZ04"
}